{
  "term_label": "Unknown molecular function",
  "gene_symbol": "DNAJC25",
  "term_id": "UNKNOWN:0001",
  "gene": "UniProtKB:Q9H1X3",
  "gene_name": "DnaJ homolog subfamily C member 25"
}